{
  "term_label": "tRNA binding",
  "term_id": "GO:0000049",
  "gene_symbol": "TRMT10A",
  "gene": "UniProtKB:Q8TBZ6",
  "gene_name": "tRNA methyltransferase 10 homolog A"
}